{
  "term_id": "GO:0005886",
  "term_label": "plasma membrane",
  "gene": "UniProtKB:Q6QEF8",
  "gene_symbol": "CORO6",
  "gene_name": "Coronin-6"
}